{
  "gene_name": "Ras-related protein Rap-2b",
  "term_label": "Rap protein signal transduction",
  "gene_symbol": "RAP2B",
  "term_id": "GO:0032486",
  "gene": "UniProtKB:P61225"
}